growth hormone receptor binding [GO:0005131] (molecular function) Relationships: is a type of cytokine receptor binding [GO:0005126]; is a type of GO:0051427 Definition: Binding to a growth hormone receptor. Sources: GOC:ai Also known as: growth hormone, growth hormone receptor ligand